phosphopolyprenol glucosyltransferase activity [GO:0047272] (molecular function) Also known as: UDP-glucose:phosphopolyprenol D-glucosyltransferase activity, UDPglucose:phosphopolyprenol D-glucosyltransferase activity, UDPglucose:polyprenol monophosphate glucosyltransferase activity, uridine diphosphoglucose-polyprenol monophosphate glucosyltransferase activity Sources: EC:2.4.1.78, MetaCyc:2.4.1.78-RXN Relationships: is a type of UDP-glucosyltransferase activity [GO:0035251] Definition: Catalysis of the reaction: polyprenyl phosphate + UDP-D-glucose = polyprenylphosphate-glucose + UDP.